L-arabinose reductase (NADPH) activity [GO:0032867] (molecular function) Definition: Catalysis of the reaction: L-arabitol + NADP+ = L-arabinose + NADPH + H+. Relationships: is a type of aldose reductase (NADPH) activity [GO:0004032] Also known as: arabinose reductase activity, arabinose:NADP reductase activity, L-arabinose:NADP reductase activity References: PMID:12724380, PMID:15184173 Sources: RHEA:25229